alanyl-tRNA aminoacylation [GO:0006419] (biological process) Subtypes: mitochondrial alanyl-tRNA aminoacylation [GO:0070143], cytoplasmic alanyl-tRNA aminoacylation [GO:1990762] Sources: GOC:mcc, ISBN:0716730510 Definition: The process of coupling alanine to alanyl-tRNA, catalyzed by alanyl-tRNA synthetase. The alanyl-tRNA synthetase is a class-II synthetases. The activated amino acid is transferred to the 3'-OH group of an alanine accetping tRNA. Relationships: is a type of GO:0006418